smooth muscle contraction involved in micturition [GO:0060083] (biological process) Definition: The process leading to shortening and/or development of tension in the urinary bladder smooth muscle tissue involved in the expulsion urine from the body. References: PMID:15827347 Sources: GOC:dph Also known as: smooth muscle contraction involved in urination, urinary bladder smooth muscle contraction involved in micturition Regulation: regulated by regulation of smooth muscle contraction involved in micturition [GO:1904318]; negatively regulated by negative regulation of smooth muscle contraction involved in micturition [GO:1904319]; positively regulated by positive regulation of smooth muscle contraction involved in micturition [GO:1904320] Relationships: is a type of urinary bladder smooth muscle contraction [GO:0014832]; is part of micturition [GO:0060073]